{
  "term_id": "UNKNOWN:0001",
  "gene_symbol": "C1orf159",
  "gene": "UniProtKB:Q96HA4",
  "term_label": "Unknown molecular function",
  "gene_name": "Uncharacterized protein C1orf159"
}